positive regulation of connective tissue replacement involved in inflammatory response wound healing [GO:1904598] (biological process) Also known as: up regulation of connective tissue replacement involved in inflammatory response wound healing, up-regulation of connective tissue replacement involved in inflammatory response wound healing, upregulation of connective tissue replacement involved in inflammatory response wound healing, activation of connective tissue replacement involved in inflammatory response wound healing, activation of fibrosis during inflammatory response, positive regulation of fibrosis during inflammatory response, up regulation of fibrosis during inflammatory response, up-regulation of fibrosis during inflammatory response, upregulation of fibrosis during inflammatory response, activation of connective tissue replacement during inflammatory response, positive regulation of connective tissue replacement during inflammatory response, up regulation of connective tissue replacement during inflammatory response, up-regulation of connective tissue replacement during inflammatory response, upregulation of connective tissue replacement during inflammatory response References: PMID:18245812 Sources: GOC:TermGenie, GOC:krc, GO_REF:0000058 Relationships: is a type of regulation of connective tissue replacement involved in inflammatory response wound healing [GO:1904596]; is a type of positive regulation of connective tissue replacement [GO:1905205]; RO_0002213 connective tissue replacement involved in inflammatory response wound healing [GO:0002248] Definition: Any process that activates or increases the frequency, rate or extent of wound healing connective tissue replacement, which may be replaced with fibrotic material, that occurs as part of an inflammatory response.